{
  "term_label": "DNA binding",
  "gene_name": "Histone H2B type 1-C_E_F_G_I",
  "gene_symbol": "H2BC10",
  "term_id": "GO:0003677",
  "gene": "UniProtKB:P62807"
}